regulation of cell communication by electrical coupling involved in cardiac conduction [GO:1901844] (biological process) Relationships: is a type of GO:0010649; RO_0002211 cell communication by electrical coupling involved in cardiac conduction [GO:0086064] Subtypes: GO:1901845, GO:1901846 References: PMID:17130302 Sources: GOC:BHF, GOC:TermGenie, GOC:rl Definition: Any process that modulates the frequency, rate or extent of cell communication by electrical coupling involved in cardiac conduction.